{
  "gene_symbol": "CCDC27",
  "term_label": "Unknown molecular function",
  "term_id": "UNKNOWN:0001",
  "gene_name": "Coiled-coil domain-containing protein 27",
  "gene": "UniProtKB:Q2M243"
}